{
  "gene_name": "Histone H3.X",
  "term_label": "heterochromatin formation",
  "term_id": "GO:0031507",
  "gene": "UniProtKB:P0DPK5",
  "gene_symbol": "H3Y2"
}